catabolite repression [GO:0061984] (biological process) Definition: A process in which the presence of one nutrient source leads to a decrease in the frequency, rate, or extent of processes involved in the metabolism of other nutrient sources. Subtypes: GO:0061985, nitrogen catabolite repression of transcription [GO:0090295] Relationships: is a type of GO:0031670; negatively regulates metabolic process [GO:0008152] References: PMID:29197127, PMID:29295552 Sources: GOC:dph